{
  "term_id": "GO:0000976",
  "gene_symbol": "ZNF197",
  "term_label": "transcription cis-regulatory region binding",
  "gene_name": "Zinc finger protein 197",
  "gene": "UniProtKB:O14709"
}